mitotic DNA integrity checkpoint signaling [GO:0044774] (biological process) Subtypes: mitotic DNA replication checkpoint signaling [GO:0033314], mitotic DNA damage checkpoint signaling [GO:0044773] Definition: A signaling process that controls cell cycle progression in response to changes in DNA structure by monitoring the integrity of the DNA during mitosis. The DNA integrity checkpoint begins with detection of DNA damage, defects in DNA structure or DNA replication, and ends with signal transduction. Relationships: is a type of mitotic cell cycle checkpoint signaling [GO:0007093]; is a type of DNA integrity checkpoint signaling [GO:0031570] Also known as: intracellular signal transduction involved in mitotic cell cycle G2/M transition decatenation checkpoint, intracellular signal transduction involved in topo II checkpoint, intracellular signal transduction pathway involved in mitotic DNA integrity checkpoint, intracellular signaling cascade involved in mitotic DNA integrity checkpoint, intracellular signaling cascade involved in mitotic cell cycle G2/M transition decatenation checkpoint, intracellular signaling cascade involved in topo II checkpoint, intracellular signaling chain involved in mitotic DNA integrity checkpoint, intracellular signaling chain involved in mitotic cell cycle G2/M transition decatenation checkpoint, intracellular signaling pathway involved in mitotic DNA integrity checkpoint, mitotic DNA integrity checkpoint, mitotic cell cycle G2/M transition decatenation checkpoint, signal transduction involved in mitotic DNA integrity checkpoint, intracellular signal transduction pathway involved in mitotic cell cycle G2/M transition decatenation checkpoint, intracellular signal transduction pathway involved in topo II checkpoint, intracellular signal transduction pathway involved in topoisomerase II checkpoint, intracellular signaling pathway involved in topo II checkpoint, intracellular signaling pathway involved in mitotic cell cycle G2/M transition decatenation checkpoint, intracellular signaling pathway involved in topoisomerase II checkpoint, signal transduction via intracellular signaling cascade involved in mitotic cell cycle G2/M transition decatenation checkpoint, signal transduction via intracellular signaling cascade involved in topo II checkpoint Sources: GOC:mtg_cell_cycle